MBF transcription complex assembly [GO:0120185] (biological process) Relationships: is a type of protein-containing complex assembly [GO:0065003] Definition: The aggregation, arrangement and bonding together of a set of components to form an MBF transcription complex. Also known as: DSC1 transcription factor complex assembly, MBF complex assembly, Mlu1-box binding factor assembly References: PMID:9303312